histone H3S10 kinase activity [GO:0035175] (MF) Relationships: is a type of protein serine/threonine kinase activity [GO:0004674]; is a type of histone H3 kinase activity [GO:0140996] References: PMID:15041176 Sources: GOC:bf Also known as: histone kinase activity (H3-S10 specific), histone serine kinase activity (H3-S10 specific), histone-serine kinase activity (H3-S10 specific) Note: Comment: Note that the residue position corresponds to the canonical human H3 histone (UniProtKB:P84243); this residue is conserved across all eukaryotes. Residue 1 is the first residue following removal of the initiating Methionine (Met). Note that each histone is encoded by multiple genes, and sequences may vary across different genes within an organism. Definition: Catalysis of the reaction: histone H3-serine (position 10) + ATP = histone H3-phosphoserine (position 10) + ADP. This reaction is the addition of a phosphate group to the serine residue at position 10 of histone H3.